{
  "term_id": "UNKNOWN:0002",
  "gene": "UniProtKB:P0DMW2",
  "gene_name": "NLR family pyrin domain-containing protein 2B",
  "term_label": "Unknown biological process",
  "gene_symbol": "NLRP2B"
}